{
  "term_label": "cytoplasmic stress granule",
  "gene_name": "La-related protein 1",
  "gene_symbol": "LARP1",
  "gene": "UniProtKB:Q6PKG0",
  "term_id": "GO:0010494"
}